{
  "term_label": "steroid Delta-isomerase activity",
  "gene_name": "3-beta-hydroxysteroid-Delta(8),Delta(7)-isomerase",
  "gene_symbol": "EBP",
  "term_id": "GO:0004769",
  "gene": "UniProtKB:Q15125"
}